{
  "gene": "UniProtKB:Q9Y6X8",
  "term_label": "regulation of transcription by RNA polymerase II",
  "term_id": "GO:0006357",
  "gene_name": "Zinc fingers and homeoboxes protein 2",
  "gene_symbol": "ZHX2"
}